transporter complex [GO:1990351] (cellular component) Relationships: is a type of protein-containing complex [GO:0032991] Note: An example of this is GTR1 in human (UniProt symbol P11166) in PMID:15449578 (inferred from direct assay). References: PMID:15449578 Sources: GOC:bhm Subtypes: tripartite ATP-independent periplasmic transporter complex [GO:0031317], GO:0061852, lipopolysaccharide transport system [GO:0062051], transmembrane transporter complex [GO:1902495], phosphatidylinositol transporter complex [GO:1902556], glucose transporter complex [GO:1990350], GO:1990429, phospholipid-translocating ATPase complex [GO:1990531] Definition: A protein complex facilitating transport of molecules (proteins, small molecules, nucleic acids) into, out of or within a cell, or between cells.